anaerobic rhamnose catabolic process [GO:0019304] (biological process) Definition: The chemical reactions and pathways resulting in the breakdown of rhamnose, the hexose 6-deoxy-L-mannose, that occurs in the absence of oxygen. Also known as: anaerobic rhamnose breakdown, anaerobic rhamnose catabolism, anaerobic rhamnose degradation Sources: GOC:ai Relationships: is a type of rhamnose catabolic process [GO:0019301]